cellular response to cyclopentenone [GO:0071410] (biological process) Relationships: is_a response to cyclopentenone [GO:0010583] Sources: GOC:mah Definition: Any process that results in a change in state or activity of a cell (in terms of movement, secretion, enzyme production, gene expression, etc.) as a result of a cyclopentenone stimulus. Cyclopentenones are oxylipins derived from polyunsaturated fatty acids. They are structurally similar to jasmonic acid, but contain a reactive unsaturated carbonyl structure in the cyclo-ring. Cyclopentenones include phytoprostanes and 12-oxo-phytodienoic acid.